glomerular epithelial cell development [GO:0072310] (biological process) Definition: The process whose specific outcome is the progression of a glomerular epithelial cell over time, from its formation to the mature structure. Glomerular epithelial cells are specialized epithelial cells that form part of the glomerulus; there are two types, glomerular parietal epithelial cells and glomerular visceral epithelial cells. Sources: GOC:mtg_kidney_jan10 Relationships: is a type of epithelial cell development [GO:0002064]; is part of glomerular epithelial cell differentiation [GO:0072311] Subtypes: mesonephric glomerular epithelial cell development [GO:0061251], GO:0072015, glomerular parietal epithelial cell development [GO:0072016], GO:0072313